3-oxo-5-alpha-steroid 4-dehydrogenase (NADP+) activity [GO:0047751] (molecular function) Sources: RHEA:54384 Relationships: is a type of GO:0003865; is a type of enone reductase activity [GO:0035671] Definition: Catalysis of the reaction: 3-oxo-5alpha-steroid + NADP+ = a 3-oxo-delta(4)-steroid + H+ + NADPH. Also known as: 3-oxosteroid delta4-dehydrogenase, steroid 5alpha-hydrogenase activity, steroid 5alpha-reductase, sterol 5-alpha reductase activity, cholestenone 5-alpha-reductase activity, cholestenone 5a-reductase activity, cholestenone 5alpha-reductase activity, progesterone 5-alpha-reductase activity, testosterone 5alpha-reductase, testosterone delta4-hydrogenase activity, 3-oxosteroid 5alpha-reductase activity